response to wortmannin [GO:1904567] (biological process) References: PMID:20629186 Sources: GOC:TermGenie, GO_REF:0000071 Definition: Any process that results in a change in state or activity of a cell or an organism (in terms of movement, secretion, enzyme production, gene expression, etc.) as a result of a wortmannin stimulus. Also known as: response to wartmannin Subtypes: cellular response to wortmannin [GO:1904568] Relationships: is a type of response to ketone [GO:1901654]